{
  "term_label": "cytosolic small ribosomal subunit",
  "gene": "UniProtKB:P62081",
  "term_id": "GO:0022627",
  "gene_name": "Small ribosomal subunit protein eS7",
  "gene_symbol": "RPS7"
}